antigen processing and presentation of endogenous peptide antigen via MHC class II [GO:0002491] (biological process) Definition: The process in which an antigen-presenting cell expresses a peptide antigen of endogenous origin on its cell surface in association with an MHC class II protein complex. The peptide antigen is typically, but not always, processed from a whole protein. References: PMID:15531770, PMID:16181338 Sources: GOC:add Also known as: endogenous peptide antigen processing and presentation via MHC class II Relationships: is a type of antigen processing and presentation of endogenous peptide antigen [GO:0002483]; is a type of antigen processing and presentation of peptide antigen via MHC class II [GO:0002495]